3-oxoacyl-[acyl-carrier-protein] reductase (NADPH) activity [GO:0004316] (molecular function) Definition: Catalysis of the reaction: (3R)-3-hydroxyacyl-[acyl-carrier protein] + NADP+ = 3-oxoacyl-[acyl-carrier protein] + NADPH + H+. Sources: RHEA:17397 Also known as: 3-oxoacyl-ACP reductase activity, 3-oxoacyl-[acyl-carrier protein] reductase activity, (3R)-3-hydroxyacyl-acyl-carrier-protein:NADP+ oxidoreductase activity, 3-ketoacyl acyl carrier protein reductase activity, 3-oxoacyl-ACPreductase activity, 3-oxoacyl-acyl-carrier-protein reductase activity, NADPH-specific 3-oxoacyl-acylcarrier proteinreductase activity, beta-ketoacyl acyl carrier protein (ACP) reductase activity, beta-ketoacyl reductase activity, beta-ketoacyl thioester reductase activity, beta-ketoacyl-ACP reductase activity, beta-ketoacyl-acyl carrier protein reductase activity, beta-ketoacyl-acyl-carrier protein(ACP) reductase activity Relationships: is a type of GO:0016616